{
  "term_label": "cytokine activity",
  "gene": "UniProtKB:Q9NPH9",
  "term_id": "GO:0005125",
  "gene_symbol": "IL26",
  "gene_name": "Interleukin-26"
}